{
  "term_label": "protein kinase regulator activity",
  "gene": "UniProtKB:P67870",
  "gene_symbol": "CSNK2B",
  "gene_name": "Casein kinase II subunit beta",
  "term_id": "GO:0019887"
}